{
  "gene_name": "Protein phosphatase 1 regulatory subunit 36",
  "gene": "UniProtKB:Q96LQ0",
  "gene_symbol": "PPP1R36",
  "term_label": "Unknown molecular function",
  "term_id": "UNKNOWN:0001"
}